{
  "gene_name": "Cytosolic 5'-nucleotidase 1A",
  "gene_symbol": "NT5C1A",
  "gene": "UniProtKB:Q9BXI3",
  "term_id": "GO:0046085",
  "term_label": "adenosine metabolic process"
}